{
  "term_id": "GO:0004984",
  "gene_symbol": "OR2B6",
  "term_label": "olfactory receptor activity",
  "gene_name": "Olfactory receptor 2B6",
  "gene": "UniProtKB:P58173"
}